{
  "gene_name": "Histidine ammonia-lyase",
  "gene_symbol": "HAL",
  "term_id": "GO:0004397",
  "gene": "UniProtKB:P42357",
  "term_label": "histidine ammonia-lyase activity"
}